aldehyde dehydrogenase (quinone) activity [GO:0047113] (molecular function) Sources: RHEA:13881 Also known as: aldehyde dehydrogenase (acceptor) activity, aldehyde dehydrogenase (pyrroloquinoline-quinone), aldehyde:(pyrroloquinoline-quinone) oxidoreductase activity Relationships: is a type of oxidoreductase activity, acting on the aldehyde or oxo group of donors [GO:0016903] Definition: Catalysis of the reaction: a quinone + an aldehyde + H2O = a carboxylate + a quinol + H+.